{
  "gene_name": "Armadillo repeat-containing X-linked protein 1",
  "gene_symbol": "ARMCX1",
  "term_label": "mitochondrion",
  "term_id": "GO:0005739",
  "gene": "UniProtKB:Q9P291"
}